{
  "gene_symbol": "PROCR",
  "gene": "UniProtKB:Q9UNN8",
  "gene_name": "Endothelial protein C receptor",
  "term_label": "extracellular space",
  "term_id": "GO:0005615"
}